short-chain fatty acid transport [GO:0015912] (biological process) Note: While there is not universal consensus on the lengths of short-, medium-, long- and very-long-chain fatty acids, the GO uses the definitions in ChEBI (see CHEBI:26666, CHEBI:59554, CHEBI:15904 and CHEBI:27283). Definition: The directed movement of short-chain fatty acids into, out of or within a cell, or between cells, by means of some agent such as a transporter or pore. A short-chain fatty acid has an aliphatic tail containing fewer than 6 carbons. Sources: GOC:ai Subtypes: short-chain fatty acid transmembrane transport [GO:0015913] Relationships: is a type of fatty acid transport [GO:0015908]